{
  "gene_name": "Putative fatty acid-binding protein 5-like protein 3",
  "gene": "UniProtKB:A8MUU1",
  "term_label": "fatty acid binding",
  "term_id": "GO:0005504",
  "gene_symbol": "FABP5P3"
}